regulation of gamma-delta T cell activation [GO:0046643] (biological process) Definition: Any process that modulates the frequency, rate or extent of gamma-delta T cell activation. Sources: GOC:ai Also known as: regulation of gamma-delta T lymphocyte activation, regulation of gamma-delta T-cell activation, regulation of gamma-delta T-lymphocyte activation Relationships: is a type of regulation of T cell activation [GO:0050863]; regulates gamma-delta T cell activation [GO:0046629] Subtypes: GO:0045586, negative regulation of gamma-delta T cell activation [GO:0046644], positive regulation of gamma-delta T cell activation [GO:0046645], GO:0046646, regulation of gamma-delta T cell activation involved in immune response [GO:2001191]